{
  "gene_symbol": "TRPM3",
  "term_id": "GO:0006816",
  "gene": "UniProtKB:Q9HCF6",
  "gene_name": "Transient receptor potential cation channel subfamily M member 3",
  "term_label": "calcium ion transport"
}